{
  "gene_name": "Otogelin-like protein",
  "term_id": "UNKNOWN:0002",
  "gene": "UniProtKB:Q3ZCN5",
  "term_label": "Unknown biological process",
  "gene_symbol": "OTOGL"
}